{
  "gene_name": "Putative uncharacterized protein encoded by LINC00526",
  "gene": "UniProtKB:Q96FQ7",
  "gene_symbol": "LINC00526",
  "term_id": "UNKNOWN:0002",
  "term_label": "Unknown biological process"
}